{
  "term_id": "GO:0033363",
  "gene_name": "Serglycin",
  "gene_symbol": "SRGN",
  "term_label": "secretory granule organization",
  "gene": "UniProtKB:P10124"
}